{
  "term_label": "guanyl-nucleotide exchange factor activity",
  "gene_symbol": "CYTH2",
  "term_id": "GO:0005085",
  "gene": "UniProtKB:Q99418",
  "gene_name": "Cytohesin-2"
}